{
  "term_id": "GO:0000978",
  "gene": "UniProtKB:Q9H6I2",
  "gene_name": "Transcription factor SOX-17",
  "term_label": "RNA polymerase II cis-regulatory region sequence-specific DNA binding",
  "gene_symbol": "SOX17"
}